{
  "term_label": "protein-macromolecule adaptor activity",
  "gene_name": "Enhancer of polycomb homolog 2",
  "gene_symbol": "EPC2",
  "gene": "UniProtKB:Q52LR7",
  "term_id": "GO:0030674"
}